{
  "term_id": "GO:0005634",
  "gene_name": "Calretinin",
  "gene_symbol": "CALB2",
  "gene": "UniProtKB:P22676",
  "term_label": "nucleus"
}